negative regulation of interleukin-4-mediated signaling pathway [GO:1902215] (biological process) Relationships: is a type of negative regulation of cytokine-mediated signaling pathway [GO:0001960]; is a type of GO:1902214; negatively regulates interleukin-4-mediated signaling pathway [GO:0035771] Also known as: down regulation of IL-4-mediated signaling pathway, down regulation of interleukin-4-mediated signaling pathway, down regulation of interleukin-4-mediated signalling pathway, down-regulation of IL-4-mediated signaling pathway, down-regulation of interleukin-4-mediated signaling pathway, down-regulation of interleukin-4-mediated signalling pathway, downregulation of IL-4-mediated signaling pathway, downregulation of interleukin-4-mediated signaling pathway, downregulation of interleukin-4-mediated signalling pathway, negative regulation of IL-4-mediated signaling pathway, negative regulation of interleukin-4-mediated signalling pathway, inhibition of IL-4-mediated signaling pathway, inhibition of interleukin-4-mediated signaling pathway, inhibition of interleukin-4-mediated signalling pathway References: PMID:17210636 Sources: GOC:TermGenie Definition: Any process that stops, prevents or reduces the frequency, rate or extent of interleukin-4-mediated signaling pathway.